{
  "term_id": "GO:0034237",
  "term_label": "protein kinase A regulatory subunit binding",
  "gene_symbol": "PRKACA",
  "gene_name": "cAMP-dependent protein kinase catalytic subunit alpha",
  "gene": "UniProtKB:P17612"
}